{
  "gene_symbol": "RNGTT",
  "gene_name": "mRNA-capping enzyme",
  "term_id": "GO:0006370",
  "gene": "UniProtKB:O60942",
  "term_label": "7-methylguanosine mRNA capping"
}